{
  "gene": "UniProtKB:Q9H5P4",
  "gene_name": "PDZ domain-containing protein 7",
  "term_label": "auditory receptor cell stereocilium organization",
  "gene_symbol": "PDZD7",
  "term_id": "GO:0060088"
}